{
  "term_id": "UNKNOWN:0001",
  "gene": "UniProtKB:Q86Y30",
  "term_label": "Unknown molecular function",
  "gene_symbol": "BAGE2",
  "gene_name": "B melanoma antigen 2"
}